{
  "term_id": "UNKNOWN:0001",
  "term_label": "Unknown molecular function",
  "gene_symbol": "TSPAN16",
  "gene": "UniProtKB:Q9UKR8",
  "gene_name": "Tetraspanin-16"
}